metallo-sulfur cluster assembly [GO:0031163] (biological process) Also known as: metal-sulfur cluster assembly, metallo-sulphur cluster assembly, metallo-sulfur cluster biosynthesis Sources: GOC:jl, GOC:mah, GOC:pde, GOC:vw Relationships: is a type of cellular component assembly [GO:0022607] Definition: The incorporation of a metal and exogenous sulfur into a metallo-sulfur cluster. Subtypes: iron-sulfur cluster assembly [GO:0016226]